{
  "term_label": "nucleus",
  "term_id": "GO:0005634",
  "gene": "UniProtKB:P55072",
  "gene_symbol": "VCP",
  "gene_name": "Transitional endoplasmic reticulum ATPase"
}